complex of collagen trimers [GO:0098644] (cellular component) Sources: GOC:dos Also known as: Supramolecular aggregate of collagen, Supramolecular collagen assembly Relationships: is a type of supramolecular complex [GO:0099080]; is part of extracellular matrix [GO:0031012]; has part GO:0005581 Subtypes: fibrillar collagen [GO:0098643], collagen network [GO:0098645], collagen beaded filament [GO:0098647], collagen anchoring fibril [GO:0098648], GO:0140153 Definition: A complex of collagen trimers such as a fibril or collagen network.